ATP-gated ion channel activity [GO:0035381] (molecular function) Sources: GOC:bf Relationships: is a type of ligand-gated channel activity [GO:0022834] Definition: Enables the transmembrane transfer of an ion by a channel that opens when ATP has been bound by the channel complex or one of its constituent parts. Subtypes: extracellularly ATP-gated monoatomic cation channel activity [GO:0004931], mitochondrial ATP-gated potassium channel activity [GO:0062156], intracellularly ATP-gated ion channel activity [GO:0099142]